creatine kinase complex [GO:0002185] (cellular component) Definition: A protein complex having creatine kinase activity. Sources: GOC:hjd Subtypes: cytosolic creatine kinase complex [GO:0002186], mitochondrial creatine kinase complex [GO:0002187] Relationships: is a type of transferase complex, transferring phosphorus-containing groups [GO:0061695]